positive regulation of ecdysteroid biosynthetic process [GO:0045998] (biological process) Definition: Any process that activates or increases the frequency, rate or extent of the chemical reactions and pathways resulting in the formation of ecdysteroids. Sources: GOC:go_curators Also known as: positive regulation of ecdysteroid anabolism, positive regulation of ecdysteroid biosynthesis, positive regulation of ecdysteroid formation, positive regulation of ecdysteroid synthesis, up regulation of ecdysteroid biosynthetic process, up-regulation of ecdysteroid biosynthetic process, upregulation of ecdysteroid biosynthetic process, activation of ecdysteroid biosynthetic process, stimulation of ecdysteroid biosynthetic process Relationships: is a type of regulation of ecdysteroid biosynthetic process [GO:0007554]; is a type of positive regulation of small molecule metabolic process [GO:0062013]; is a type of positive regulation of steroid hormone biosynthetic process [GO:0090031]; positively regulates ecdysteroid biosynthetic process [GO:0045456]